{
  "term_id": "GO:0050853",
  "gene_symbol": "TEC",
  "term_label": "B cell receptor signaling pathway",
  "gene": "UniProtKB:P42680",
  "gene_name": "Tyrosine-protein kinase Tec"
}